{
  "term_id": "GO:0016226",
  "gene_name": "Frataxin, mitochondrial",
  "term_label": "iron-sulfur cluster assembly",
  "gene_symbol": "FXN",
  "gene": "UniProtKB:Q16595"
}